{
  "gene_symbol": "FAM169A",
  "term_id": "UNKNOWN:0002",
  "gene_name": "Soluble lamin-associated protein of 75 kDa",
  "gene": "UniProtKB:Q9Y6X4",
  "term_label": "Unknown biological process"
}